{
  "term_label": "Unknown molecular function",
  "gene_symbol": "HERV-K104",
  "gene_name": "Endogenous retrovirus group K member 104 Pro protein",
  "term_id": "UNKNOWN:0001",
  "gene": "UniProtKB:P63124"
}